{
  "term_label": "actin cytoskeleton organization",
  "term_id": "GO:0030036",
  "gene_symbol": "WASF3",
  "gene_name": "Actin-binding protein WASF3",
  "gene": "UniProtKB:Q9UPY6"
}